{
  "gene": "UniProtKB:P22466",
  "gene_symbol": "GAL",
  "gene_name": "Galanin peptides",
  "term_label": "extracellular space",
  "term_id": "GO:0005615"
}